{
  "gene_symbol": "KRT9",
  "term_label": "keratin filament",
  "gene_name": "Keratin, type I cytoskeletal 9",
  "gene": "UniProtKB:P35527",
  "term_id": "GO:0045095"
}